{
  "term_id": "GO:0007166",
  "term_label": "cell surface receptor signaling pathway",
  "gene_name": "T cell receptor beta variable 2",
  "gene_symbol": "TRBV2",
  "gene": "UniProtKB:A0A1B0GX68"
}